{
  "term_label": "Unknown molecular function",
  "gene_symbol": "ADAMTSL5",
  "term_id": "UNKNOWN:0001",
  "gene_name": "ADAMTS-like protein 5",
  "gene": "UniProtKB:Q6ZMM2"
}